6-hydroxycyclohex-1-ene-1-carboxyl-CoA hydratase activity [GO:0018807] (molecular function) Relationships: is_a GO:0016822 Sources: UM-BBD_reactionID:r0204 Definition: Catalysis of the reaction: 6-hydroxycyclohex-1-ene-1-carboxyl-CoA + H2O = 2,6-dihydroxycyclohexane-1-carboxyl-CoA.